{
  "gene": "UniProtKB:Q9UKA4",
  "term_label": "protein kinase A binding",
  "term_id": "GO:0051018",
  "gene_name": "A-kinase anchor protein 11",
  "gene_symbol": "AKAP11"
}